Hulle cell development [GO:0070792] (biological process) References: PMID:19210625 Regulation: regulated by regulation of Hulle cell development [GO:0070808]; negatively regulated by negative regulation of Hulle cell development [GO:0070809]; positively regulated by positive regulation of Hulle cell development [GO:0070810] Relationships: is a type of developmental process involved in reproduction [GO:0003006]; is a type of cell development [GO:0048468]; is part of GO:0070791 Also known as: Huelle cell development, Hulle cell formation Definition: The process whose specific outcome is the progression of Hulle cells over time, from their formation to the mature structures. Hulle cells are specialized multinucleate cells that originate from a nest-like aggregation of hyphae during sexual development and serve as nurse cells to the developing cleistothecium, or fruiting body.